positive regulation of interleukin-7 production [GO:0032756] (biological process) Sources: GOC:mah Also known as: positive regulation of IL-7 production, up regulation of interleukin-7 production, up-regulation of interleukin-7 production, upregulation of interleukin-7 production, activation of interleukin-7 production, positive regulation of interleukin-7 biosynthetic process, positive regulation of interleukin-7 secretion, stimulation of interleukin-7 production Relationships: is a type of positive regulation of cytokine production [GO:0001819]; is a type of regulation of interleukin-7 production [GO:0032676]; RO_0002213 GO:0032636 Definition: Any process that activates or increases the frequency, rate, or extent of interleukin-7 production.